molybdopterin adenylyltransferase complex [GO:1990133] (cellular component) Relationships: is a type of adenylyltransferase complex [GO:1902503]; is part of cytosol [GO:0005829] Definition: A heterotetrameric protein complex which adenylates two molecules of the sulfur carrier subunit of the molybdopterin cofactor synthase using ATP as part of molybdopterin cofactor (Moco) biosynthesis. In E. coli the subunits are MoeB and MoaD; in human the subunits are MOCS3 and MOCS2A. Moco biosynthesis and its constituent molecules are evolutionarily conserved. Also known as: MPT adenylyltransferase complex, molybdopterin cofactor (Moco) biosynthesis adenylyltransferase complex References: PMID:11713534, PMID:16669776, PMID:18491921 Sources: GOC:bhm